{
  "gene": "UniProtKB:Q92947",
  "term_label": "glutaryl-CoA dehydrogenase activity",
  "gene_name": "Glutaryl-CoA dehydrogenase, mitochondrial",
  "gene_symbol": "GCDH",
  "term_id": "GO:0004361"
}